protein tag activity [GO:0031386] (molecular function) Relationships: is a type of molecular tag activity [GO:0141047] Also known as: covalent modifier, protein tag, ubiquitin-like protein modifier, protein tagging activity, ubiquitin References: PMID:19028679, PMID:20054389, PMID:6305978 Sources: GOC:dos Note: Use this term to annotate conjugated tags, not for conjugating enzymes. At the time of writing, all known gene products with this activity are ubiquitin-like, either based on overall sequence similarity or the presence of common motifs and structures. Definition: A molecular function exhibited by a protein that is covalently attached (AKA tagged or conjugated) to another protein where it acts as a marker, recognized by the cellular apparatus to target the tagged protein for some cellular process such as modification, sequestration, transport or degradation.